{
  "gene_symbol": "RAD50",
  "gene": "UniProtKB:Q92878",
  "term_label": "Mre11 complex",
  "term_id": "GO:0030870",
  "gene_name": "DNA repair protein RAD50"
}